{
  "gene_symbol": "GOLGA8IP",
  "gene": "UniProtKB:A6NC78",
  "gene_name": "Putative golgin subfamily A member 8I",
  "term_id": "GO:0000137",
  "term_label": "Golgi cis cisterna"
}